{
  "gene": "UniProtKB:Q92900",
  "gene_symbol": "UPF1",
  "term_label": "cytoplasm",
  "gene_name": "Regulator of nonsense transcripts 1",
  "term_id": "GO:0005737"
}